amylopectin biosynthetic process [GO:0010021] (BP) Sources: ISBN:0943088399 Also known as: amylopectin anabolism, amylopectin biosynthesis, amylopectin formation, amylopectin synthesis Relationships: is a type of macromolecule biosynthetic process [GO:0009059]; is a type of carbohydrate derivative biosynthetic process [GO:1901137]; is a type of amylopectin metabolic process [GO:2000896] Definition: The chemical reactions and pathways resulting in the formation of amylopectin, the (1->4) linked alpha glucose units with alpha-(1->6) linkages.